{
  "term_id": "GO:0003747",
  "gene": "UniProtKB:P15170",
  "gene_symbol": "GSPT1",
  "term_label": "translation release factor activity",
  "gene_name": "Eukaryotic peptide chain release factor GTP-binding subunit ERF3A"
}